{
  "gene": "UniProtKB:P62318",
  "term_label": "commitment complex",
  "term_id": "GO:0000243",
  "gene_name": "Small nuclear ribonucleoprotein Sm D3",
  "gene_symbol": "SNRPD3"
}